{
  "gene": "UniProtKB:Q9UC06",
  "gene_name": "Zinc finger protein 70",
  "term_label": "nucleus",
  "gene_symbol": "ZNF70",
  "term_id": "GO:0005634"
}